regulation of carbon utilization [GO:0043609] (biological process) Definition: Any process that modulates the frequency, rate, or extent of carbon utilization. Sources: GOC:jl Relationships: is a type of GO:0032107; regulates carbon utilization [GO:0015976]